{
  "gene": "UniProtKB:Q03181",
  "term_id": "GO:0030154",
  "gene_name": "Peroxisome proliferator-activated receptor delta",
  "gene_symbol": "PPARD",
  "term_label": "cell differentiation"
}